{
  "gene_symbol": "OR4X2",
  "term_id": "GO:0004984",
  "term_label": "olfactory receptor activity",
  "gene": "UniProtKB:Q8NGF9",
  "gene_name": "Olfactory receptor 4X2"
}